{
  "gene_symbol": "APOA5",
  "gene": "UniProtKB:Q6Q788",
  "term_label": "phospholipid binding",
  "term_id": "GO:0005543",
  "gene_name": "Apolipoprotein A-V"
}